aminomuconate-semialdehyde dehydrogenase activity [GO:0047102] (molecular function) Sources: EC:1.2.1.32, MetaCyc:1.2.1.32-RXN Definition: Catalysis of the reaction: H2O + NAD+ + 2-aminomuconate semialdehyde = NADH + 2-amino-muconate. Also known as: 2-aminomuconate semialdehyde dehydrogenase activity, 2-aminomuconate-6-semialdehyde:NAD+ 6-oxidoreductase activity, 2-hydroxymuconate semialdehyde dehydrogenase activity, 2-hydroxymuconic acid semialdehyde dehydrogenase activity, 2-hydroxymuconic semialdehyde dehydrogenase activity, alpha-aminomuconic epsilon-semialdehyde dehydrogenase activity, alpha-hydroxymuconic epsilon-semialdehyde dehydrogenase activity Relationships: is a type of oxidoreductase activity, acting on the aldehyde or oxo group of donors, NAD or NADP as acceptor [GO:0016620]